{
  "gene": "UniProtKB:O95169",
  "term_id": "GO:0045271",
  "gene_symbol": "NDUFB8",
  "term_label": "respiratory chain complex I",
  "gene_name": "NADH dehydrogenase [ubiquinone] 1 beta subcomplex subunit 8, mitochondrial"
}